regulation of mechanoreceptor differentiation [GO:0045631] (biological process) Sources: GOC:go_curators Subtypes: GO:0045632, positive regulation of mechanoreceptor differentiation [GO:0045633], regulation of inner ear receptor cell differentiation [GO:2000980] Relationships: is a type of regulation of neuron differentiation [GO:0045664]; regulates mechanoreceptor differentiation [GO:0042490] Definition: Any process that modulates the frequency, rate or extent of mechanoreceptor differentiation.